{
  "term_label": "Unknown biological process",
  "term_id": "UNKNOWN:0002",
  "gene_symbol": "RDM1",
  "gene": "UniProtKB:Q8NG50",
  "gene_name": "RAD52 motif-containing protein 1"
}